{
  "term_id": "GO:0043022",
  "term_label": "ribosome binding",
  "gene_name": "Cytoplasmic polyadenylation element-binding protein 4",
  "gene_symbol": "CPEB4",
  "gene": "UniProtKB:Q17RY0"
}